microtubule minus-end [GO:0036449] (cellular component) Definition: The end of a microtubule that does not preferentially grow (polymerize). Subtypes: cytoplasmic microtubule minus-end [GO:0062194] References: PMID:23169647 Sources: GOC:lb Relationships: is_a microtubule end [GO:1990752] Also known as: microtubule minus end